{
  "term_id": "GO:0043539",
  "term_label": "protein serine/threonine kinase activator activity",
  "gene_symbol": "CAB39L",
  "gene": "UniProtKB:Q9H9S4",
  "gene_name": "Calcium-binding protein 39-like"
}